{
  "gene_symbol": "GPR22",
  "gene_name": "G-protein coupled receptor 22",
  "gene": "UniProtKB:Q99680",
  "term_label": "plasma membrane",
  "term_id": "GO:0005886"
}